{
  "gene_symbol": "PLCE1",
  "gene": "UniProtKB:Q9P212",
  "term_id": "GO:0048015",
  "gene_name": "1-phosphatidylinositol 4,5-bisphosphate phosphodiesterase epsilon-1",
  "term_label": "phosphatidylinositol-mediated signaling"
}